regulation of ecdysone receptor signaling pathway [GO:0120141] (biological process) Relationships: is a type of GO:0033143; is_a regulation of cellular response to alcohol [GO:1905957]; regulates GO:0035076 Also known as: regulation of ecdysone receptor-mediated signaling pathway Definition: Any process that modulates the frequency, rate or extent of the activity of any ecdysone receptor signaling pathway. References: PMID:23072462 Sources: GOC:ha Subtypes: positive regulation of ecdysone receptor signaling pathway [GO:0120142], negative regulation of ecdysone receptor signaling pathway [GO:0120143]